{
  "term_id": "GO:0035721",
  "term_label": "intraciliary retrograde transport",
  "gene_name": "WD repeat-containing protein 35",
  "gene_symbol": "WDR35",
  "gene": "UniProtKB:Q9P2L0"
}